{
  "term_id": "GO:0032807",
  "gene_name": "DNA ligase 4",
  "gene_symbol": "LIG4",
  "term_label": "DNA ligase IV complex",
  "gene": "UniProtKB:P49917"
}